{
  "term_id": "GO:0004489",
  "gene_symbol": "MTHFR",
  "gene_name": "Methylenetetrahydrofolate reductase (NADPH)",
  "gene": "UniProtKB:P42898",
  "term_label": "methylenetetrahydrofolate reductase [NAD(P)H] activity"
}